{
  "gene_name": "Glycine N-acyltransferase-like protein 2",
  "term_label": "glycine N-acyltransferase activity",
  "term_id": "GO:0047961",
  "gene": "UniProtKB:Q8WU03",
  "gene_symbol": "GLYATL2"
}